{
  "gene": "UniProtKB:O75290",
  "term_label": "DNA-binding transcription factor activity, RNA polymerase II-specific",
  "gene_name": "Zinc finger protein 780A",
  "term_id": "GO:0000981",
  "gene_symbol": "ZNF780A"
}